{
  "term_id": "GO:0005737",
  "gene": "UniProtKB:Q7Z6W7",
  "term_label": "cytoplasm",
  "gene_symbol": "DNAJB7",
  "gene_name": "DnaJ homolog subfamily B member 7"
}